{
  "term_id": "UNKNOWN:0001",
  "gene_name": "Cilia- and flagella-associated protein 95",
  "gene_symbol": "CFAP95",
  "gene": "UniProtKB:Q5VTT2",
  "term_label": "Unknown molecular function"
}